{
  "term_id": "GO:0003677",
  "gene_name": "Deoxyribonuclease-1-like 1",
  "gene": "UniProtKB:P49184",
  "gene_symbol": "DNASE1L1",
  "term_label": "DNA binding"
}